hydrogen selenide methyltransferase activity [GO:0098614] (molecular function) Definition: Catalysis of the reaction: S-adenosyl-L-methionine + hydrogen selenide = S-adenosyl-L-homocysteine + methaneselenol. References: PMID:14705, PMID:17988700 Relationships: is a type of methyltransferase activity [GO:0008168]